oxidoreductase activity, acting on metal ions [GO:0016722] (molecular function) Definition: Catalysis of an oxidation-reduction in which the oxidation state of metal ion is altered. Sources: GOC:mah Subtypes: ferric-chelate reductase activity [GO:0000293], oxidoreductase activity, acting on metal ions, NAD or NADP as acceptor [GO:0016723], oxidoreductase activity, acting on metal ions, oxygen as acceptor [GO:0016724], transmembrane ascorbate ferrireductase activity [GO:0140571] Relationships: is a type of oxidoreductase activity [GO:0016491] Also known as: oxidoreductase activity, oxidizing metal ions, oxidoreductase activity, reducing metal ions